{
  "term_label": "transcription cis-regulatory region binding",
  "gene_symbol": "ZNF224",
  "gene_name": "Zinc finger protein 224",
  "gene": "UniProtKB:Q9NZL3",
  "term_id": "GO:0000976"
}